{
  "gene_symbol": "GOLGA6C",
  "gene": "UniProtKB:A6NDK9",
  "term_id": "GO:0007030",
  "gene_name": "Golgin subfamily A member 6C",
  "term_label": "Golgi organization"
}